signaling receptor activity [GO:0038023] (molecular function) Subtypes: phorbol ester receptor activity [GO:0001565], GO:0001653, GO:0004879, transmembrane signaling receptor activity [GO:0004888], cell adhesion receptor activity [GO:0004895], neurotrophin receptor activity [GO:0005030], GO:0008036, photoreceptor activity [GO:0009881], GO:0015026, protein-hormone receptor activity [GO:0016500], high molecular weight B cell growth factor receptor activity [GO:0030373], urokinase plasminogen activator receptor activity [GO:0030377], neurotransmitter receptor activity [GO:0030594], pattern recognition receptor activity [GO:0038187], auxin receptor activity [GO:0038198], ethylene receptor activity [GO:0038199], leucokinin receptor activity [GO:0042071], corticotropin-releasing hormone receptor activity [GO:0043404], advanced glycation end-product receptor activity [GO:0050785], 4-hydroxybutyrate receptor activity [GO:0062124], thrombospondin receptor activity [GO:0070053], GO:0140375, carbon dioxide receptor activity [GO:0170015], cord factor receptor activity [GO:1990725] Relationships: is a type of molecular transducer activity [GO:0060089] Also known as: receptor activity, receptor activity involved in signal transduction, signalling receptor activity Sources: GOC:bf, GOC:signaling Regulation: regulated by regulation of signaling receptor activity [GO:0010469]; regulated by GO:0030545; positively regulated by signaling receptor activator activity [GO:0030546]; RO_0002212 by signaling receptor inhibitor activity [GO:0030547]; negatively regulated by negative regulation of signaling receptor activity [GO:2000272] Definition: Receiving a signal and transmitting it in the cell to initiate a change in cell activity. A signal is a physical entity or change in state that is used to transfer information in order to trigger a response.